muscle filament sliding [GO:0030049] (biological process) Relationships: is a type of actin-myosin filament sliding [GO:0033275]; is part of muscle contraction [GO:0006936] Sources: GOC:mah, GOC:mtg_muscle, ISBN:0815316194 Regulation: regulated by regulation of muscle filament sliding [GO:0032971]; negatively regulated by negative regulation of muscle filament sliding [GO:1904113]; positively regulated by positive regulation of muscle filament sliding [GO:1904114] Definition: The sliding of actin thin filaments and myosin thick filaments past each other in muscle contraction. This involves a process of interaction of myosin located on a thick filament with actin located on a thin filament. During this process ATP is split and forces are generated.